{
  "term_id": "GO:0007268",
  "gene_name": "Synaptotagmin-9",
  "gene_symbol": "SYT9",
  "term_label": "chemical synaptic transmission",
  "gene": "UniProtKB:Q86SS6"
}